{
  "term_id": "GO:0030018",
  "gene_symbol": "CASQ1",
  "gene": "UniProtKB:P31415",
  "term_label": "Z disc",
  "gene_name": "Calsequestrin-1"
}